{
  "term_id": "GO:0005634",
  "gene": "UniProtKB:P15976",
  "gene_symbol": "GATA1",
  "gene_name": "Erythroid transcription factor",
  "term_label": "nucleus"
}